trans-1,2-dihydrobenzene-1,2-diol dehydrogenase activity [GO:0047115] (molecular function) Definition: Catalysis of the reaction: NADP+ + trans-1,2-dihydrobenzene-1,2-diol = NADPH + catechol. Sources: EC:1.3.1.20, MetaCyc:1.3.1.20-RXN Also known as: dihydrodiol dehydrogenase activity, trans-1,2-dihydrobenzene-1,2-diol:NADP+ oxidoreductase activity Relationships: is a type of GO:0016628